{
  "gene": "UniProtKB:Q9UBN1",
  "term_label": "transmission of nerve impulse",
  "gene_name": "Voltage-dependent calcium channel gamma-4 subunit",
  "term_id": "GO:0019226",
  "gene_symbol": "CACNG4"
}